{
  "term_id": "GO:0005802",
  "gene": "UniProtKB:Q8N4B1",
  "gene_name": "Sesquipedalian-1",
  "term_label": "trans-Golgi network",
  "gene_symbol": "PHETA1"
}